{
  "gene_symbol": "OGFOD2",
  "gene_name": "2-oxoglutarate and iron-dependent oxygenase domain-containing protein 2",
  "term_label": "Unknown molecular function",
  "gene": "UniProtKB:Q6N063",
  "term_id": "UNKNOWN:0001"
}